{
  "term_id": "GO:0005634",
  "term_label": "nucleus",
  "gene_symbol": "ZNF77",
  "gene": "UniProtKB:Q15935",
  "gene_name": "Zinc finger protein 77"
}